{
  "term_label": "plasma membrane",
  "term_id": "GO:0005886",
  "gene": "UniProtKB:Q9H223",
  "gene_symbol": "EHD4",
  "gene_name": "EH domain-containing protein 4"
}